{
  "term_id": "GO:0005829",
  "gene_symbol": "ATG3",
  "gene": "UniProtKB:Q9NT62",
  "gene_name": "Ubiquitin-like-conjugating enzyme ATG3",
  "term_label": "cytosol"
}